pyrimidine deoxyribonucleoside triphosphate biosynthetic process [GO:0009212] (biological process) Subtypes: dUTP biosynthetic process [GO:0006229], dTTP biosynthetic process [GO:0006235], dCTP biosynthetic process [GO:0006242] Sources: GOC:go_curators, ISBN:0198506732 Also known as: pyrimidine deoxyribonucleoside triphosphate anabolism, pyrimidine deoxyribonucleoside triphosphate biosynthesis, pyrimidine deoxyribonucleoside triphosphate formation, pyrimidine deoxyribonucleoside triphosphate synthesis Definition: The chemical reactions and pathways resulting in the formation of pyrimidine deoxyribonucleoside triphosphate, a compound consisting of a pyrimidine base linked to a deoxyribose sugar esterified with triphosphate on the sugar. Relationships: is a type of pyrimidine nucleoside triphosphate biosynthetic process [GO:0009148]; is a type of pyrimidine deoxyribonucleoside triphosphate metabolic process [GO:0009211]